{
  "term_label": "regulation of synaptic transmission, glutamatergic",
  "gene": "UniProtKB:Q14831",
  "gene_symbol": "GRM7",
  "gene_name": "Metabotropic glutamate receptor 7",
  "term_id": "GO:0051966"
}